{
  "gene": "UniProtKB:Q9Y312",
  "gene_name": "Protein AAR2 homolog",
  "term_id": "UNKNOWN:0001",
  "gene_symbol": "AAR2",
  "term_label": "Unknown molecular function"
}